{
  "term_id": "UNKNOWN:0002",
  "term_label": "Unknown biological process",
  "gene": "UniProtKB:Q96A99",
  "gene_name": "Pentraxin-4",
  "gene_symbol": "PTX4"
}